{
  "gene": "UniProtKB:P24278",
  "gene_name": "Zinc finger and BTB domain-containing protein 25",
  "gene_symbol": "ZBTB25",
  "term_id": "GO:0000122",
  "term_label": "negative regulation of transcription by RNA polymerase II"
}